pyridine-containing compound catabolic process [GO:0072526] (biological process) Sources: GOC:mah Subtypes: pyridine nucleotide catabolic process [GO:0019364], quinolinate catabolic process [GO:0034213], GO:0042820, pyridine catabolic process [GO:0046221], pyridine nucleoside catabolic process [GO:0070638], GO:1901517, aspyridone B catabolic process [GO:1901520], nicotinate catabolic process [GO:1901848] Relationships: is a type of catabolic process [GO:0009056]; is_a pyridine-containing compound metabolic process [GO:0072524] Also known as: pyridine and derivative catabolic process, pyridine-containing compound breakdown, pyridine-containing compound catabolism, pyridine-containing compound degradation Definition: The chemical reactions and pathways resulting in the breakdown of a pyridine-containing compound, i.e. any compound that contains pyridine or a formal derivative thereof.